cellular response to bleomycin [GO:1904976] (biological process) Definition: Any process that results in a change in state or activity of a cell (in terms of movement, secretion, enzyme production, gene expression, etc.) as a result of a bleomycin stimulus. References: PMID:11553781 Sources: GOC:TermGenie, GO_REF:0000071 Relationships: is a type of cellular response to nitrogen compound [GO:1901699]; is a type of cellular response to oxygen-containing compound [GO:1901701]; is_a GO:1904975